response to gonadotropin [GO:0034698] (BP) Relationships: is a type of response to hormone [GO:0009725] Also known as: response to gonadotropin stimulus Definition: Any process that results in a change in state or activity of a cell or an organism (in terms of movement, secretion, enzyme production, gene expression, etc.) as a result of a gonadotropin stimulus. Sources: GOC:BHF, GOC:vk Subtypes: response to follicle-stimulating hormone [GO:0032354], response to luteinizing hormone [GO:0034699], response to human chorionic gonadotropin [GO:0044752], cellular response to gonadotropin stimulus [GO:0071371]